{
  "term_id": "GO:0002891",
  "term_label": "positive regulation of immunoglobulin mediated immune response",
  "gene_symbol": "NECTIN2",
  "gene": "UniProtKB:Q92692",
  "gene_name": "Nectin-2"
}